trypsinogen activation [GO:0032023] (biological process) Sources: GOC:mah Also known as: cleavage of trypsinogen to trypsin Definition: The proteolytic processing of trypsinogen to the active form, trypsin. Relationships: is_a zymogen activation [GO:0031638]